renal sodium ion transport [GO:0003096] (BP) Relationships: is a type of renal system process [GO:0003014]; is a type of sodium ion transport [GO:0006814] Definition: The directed movement of sodium ions (Na+) by the renal system. Sources: GOC:mtg_cardio Subtypes: GO:0070294